trunk segmentation [GO:0035290] (biological process) Relationships: is a type of segmentation [GO:0035282]; is part of blastoderm segmentation [GO:0007350] References: PMID:1360402 Definition: Partitioning of the blastoderm embryo into trunk segmental units. In Drosophila, the trunk segments include thoracic segments and abdominal segments A1 to A8.